{
  "gene": "UniProtKB:Q9NWC5",
  "gene_symbol": "TMEM45A",
  "gene_name": "Transmembrane protein 45A",
  "term_id": "UNKNOWN:0003",
  "term_label": "Unknown cellular component"
}